{
  "gene": "UniProtKB:Q3B7J2",
  "gene_name": "Glucose-fructose oxidoreductase domain-containing protein 2",
  "term_label": "Unknown molecular function",
  "term_id": "UNKNOWN:0001",
  "gene_symbol": "GFOD2"
}